{
  "gene": "UniProtKB:P09067",
  "term_label": "anterior/posterior pattern specification",
  "term_id": "GO:0009952",
  "gene_symbol": "HOXB5",
  "gene_name": "Homeobox protein Hox-B5"
}